{
  "gene_name": "Clavesin-1",
  "term_id": "GO:0007040",
  "gene": "UniProtKB:Q8IUQ0",
  "gene_symbol": "CLVS1",
  "term_label": "lysosome organization"
}